{
  "gene": "UniProtKB:A6NM76",
  "term_label": "olfactory receptor activity",
  "gene_symbol": "OR6C76",
  "gene_name": "Olfactory receptor 6C76",
  "term_id": "GO:0004984"
}